hydroxyapatite binding [GO:0046848] (molecular function) Relationships: is a type of small molecule binding [GO:0036094] References: PMID:2438276 Definition: Binding to hydroxyapatite, the calcium phosphate mineral of formula Ca10(PO4)6(OH)2 found both in rocks of nonorganic origin and as a component of bone and dentin. Also known as: hydroxylapatite binding